{
  "term_id": "GO:0045944",
  "gene": "UniProtKB:Q07869",
  "term_label": "positive regulation of transcription by RNA polymerase II",
  "gene_name": "Peroxisome proliferator-activated receptor alpha",
  "gene_symbol": "PPARA"
}